{
  "gene_symbol": "ANK3",
  "gene": "UniProtKB:Q12955",
  "term_label": "neuron projection",
  "term_id": "GO:0043005",
  "gene_name": "Ankyrin-3"
}